{
  "term_id": "GO:0005634",
  "term_label": "nucleus",
  "gene_name": "Four and a half LIM domains protein 3",
  "gene": "UniProtKB:Q13643",
  "gene_symbol": "FHL3"
}